{
  "gene_symbol": "UTS2B",
  "gene": "UniProtKB:Q765I0",
  "term_id": "GO:0001664",
  "term_label": "G protein-coupled receptor binding",
  "gene_name": "Urotensin-2B"
}